{
  "term_label": "epidermis development",
  "gene": "UniProtKB:P60985",
  "term_id": "GO:0008544",
  "gene_name": "Keratinocyte differentiation-associated protein",
  "gene_symbol": "KRTDAP"
}